{
  "gene_name": "Gamma-aminobutyric acid receptor subunit alpha-4",
  "term_id": "GO:0008503",
  "gene_symbol": "GABRA4",
  "term_label": "benzodiazepine receptor activity",
  "gene": "UniProtKB:P48169"
}